inositol-3,4,6-trisphosphate 1-kinase activity [GO:0052835] (molecular function) References: PMID:11909533 Sources: RHEA:70287 Also known as: 1D-myo-inositol-trisphosphate 1-kinase activity, IP3 1-kinase activity, inositol-trisphosphate 1-kinase activity, inositol 3,4,6-trisphosphate 1-kinase activity, Ins(3,4,6)P3 1-kinase activity, ins(3,4,6)P(3) 1-kinase activity Definition: Catalysis of the reaction: 1D-myo-inositol 3,4,6-trisphosphate + ATP = 1D-myo-inositol 1,3,4,6-tetrakisphosphate + ADP + H+. Relationships: is a type of inositol trisphosphate kinase activity [GO:0051766]